{
  "gene_symbol": "MRAP2",
  "term_id": "GO:0070996",
  "gene": "UniProtKB:Q96G30",
  "gene_name": "Melanocortin-2 receptor accessory protein 2",
  "term_label": "type 1 melanocortin receptor binding"
}